{
  "term_label": "Unknown biological process",
  "gene_name": "Lipoyltransferase 1, mitochondrial",
  "term_id": "UNKNOWN:0002",
  "gene_symbol": "LIPT1",
  "gene": "UniProtKB:Q9Y234"
}